{
  "gene_symbol": "CST8",
  "gene": "UniProtKB:O60676",
  "term_label": "cytoplasm",
  "term_id": "GO:0005737",
  "gene_name": "Cystatin-8"
}